flagellated sperm motility [GO:0030317] (biological process) References: PMID:26680031 Sources: GOC:TermGenie, GOC:cilia, GOC:krc, GO_REF:0000060 Also known as: sperm motility, sperm movement, flagellated sperm movement, sperm flagellum movement, sperm flagellum movement involved in flagellated sperm motility, sperm flagellum movement involved in flagellated sperm movement Relationships: is a type of GO:0060285; is_a cilium movement involved in cell motility [GO:0060294]; is a type of sperm motility [GO:0097722] Regulation: regulated by regulation of flagellated sperm motility [GO:1901317]; negatively regulated by negative regulation of flagellated sperm motility [GO:1901318]; positively regulated by positive regulation of flagellated sperm motility [GO:1902093] Definition: The directed, self-propelled movement of a cilium (aka flagellum) that contributes to the movement of a flagellated sperm.